{
  "term_label": "Unknown biological process",
  "term_id": "UNKNOWN:0002",
  "gene_name": "CD320 antigen",
  "gene": "UniProtKB:Q9NPF0",
  "gene_symbol": "CD320"
}